{
  "term_label": "mRNA 3'-UTR binding",
  "gene_symbol": "CPEB4",
  "gene": "UniProtKB:Q17RY0",
  "gene_name": "Cytoplasmic polyadenylation element-binding protein 4",
  "term_id": "GO:0003730"
}